{
  "gene": "UniProtKB:Q8TBB6",
  "gene_symbol": "SLC7A14",
  "gene_name": "Probable cationic amino acid transporter",
  "term_label": "plasma membrane",
  "term_id": "GO:0005886"
}